polyphosphate-glucose phosphotransferase activity [GO:0047330] (molecular function) Definition: Catalysis of the reaction: beta-D-glucose + long chain polyphosphate = glucose-6-phosphate + long chain polyphosphate. Relationships: is a type of kinase activity [GO:0016301]; is_a phosphotransferase activity, alcohol group as acceptor [GO:0016773] Sources: EC:2.7.1.63, MetaCyc:2.7.1.63-RXN Also known as: polyphosphate glucokinase activity, polyphosphate-D-(+)-glucose-6-phosphotransferase activity, polyphosphate-glucose 6-phosphotransferase activity, polyphosphate:D-glucose 6-phosphotransferase activity